casbene synthase activity [GO:0050449] (molecular function) Also known as: casbene synthetase activity, geranylgeranyl-diphosphate diphosphate-lyase (cyclizing), geranylgeranyl-diphosphate diphosphate-lyase (cyclizing, casbene-forming) Definition: Catalysis of the reaction: all-trans-geranylgeranyl diphosphate = casbene + diphosphate. Relationships: is a type of terpene synthase activity [GO:0010333] Sources: EC:4.2.3.8, RHEA:14901